meiotic DNA recombinase assembly [GO:0000707] (biological process) References: PMID:11459983 Sources: GOC:elh Definition: During meiosis, the aggregation, arrangement and bonding together of strand exchange proteins (recombinases) to form higher order oligomers on single-stranded DNA. Relationships: is a type of GO:0000730; is a type of meiosis I cell cycle process [GO:0061982] Subtypes: GO:0007146, meiotic DNA recombinase assembly involved in reciprocal meiotic recombination [GO:0010772], meiotic DNA recombinase assembly involved in meiotic gene conversion [GO:0010773]